{
  "term_label": "histone binding",
  "gene_symbol": "TSPYL6",
  "term_id": "GO:0042393",
  "gene_name": "Testis-specific Y-encoded-like protein 6",
  "gene": "UniProtKB:Q8N831"
}